{
  "term_label": "Unknown cellular component",
  "term_id": "UNKNOWN:0003",
  "gene_name": "Putative uncharacterized protein FLJ39060",
  "gene": "UniProtKB:Q8N8P6",
  "gene_symbol": "Q8N8P6"
}